{
  "term_id": "UNKNOWN:0003",
  "term_label": "Unknown cellular component",
  "gene_name": "Sec1 family domain-containing protein 2",
  "gene": "UniProtKB:Q8WU76",
  "gene_symbol": "SCFD2"
}